{
  "gene_symbol": "TRAJ34",
  "term_label": "Unknown molecular function",
  "gene": "UniProtKB:A0N4X5",
  "gene_name": "HCG2039756 (Fragment)",
  "term_id": "UNKNOWN:0001"
}